{
  "term_id": "GO:0004674",
  "gene_name": "Serine_threonine-protein kinase N3",
  "gene_symbol": "PKN3",
  "term_label": "protein serine/threonine kinase activity",
  "gene": "UniProtKB:Q6P5Z2"
}